{
  "gene_name": "Bone marrow stromal antigen 2",
  "gene": "UniProtKB:Q10589",
  "gene_symbol": "BST2",
  "term_id": "GO:0005794",
  "term_label": "Golgi apparatus"
}